{
  "term_id": "GO:0035267",
  "gene": "UniProtKB:O95619",
  "term_label": "NuA4 histone acetyltransferase complex",
  "gene_name": "YEATS domain-containing protein 4",
  "gene_symbol": "YEATS4"
}